{
  "gene_symbol": "CHRNA7",
  "term_id": "GO:0043005",
  "term_label": "neuron projection",
  "gene": "UniProtKB:P36544",
  "gene_name": "Neuronal acetylcholine receptor subunit alpha-7"
}